{
  "gene_name": "Zinc finger protein 732",
  "term_id": "GO:0000978",
  "term_label": "RNA polymerase II cis-regulatory region sequence-specific DNA binding",
  "gene_symbol": "ZNF732",
  "gene": "UniProtKB:B4DXR9"
}